phosphoribosylglycinamide formyltransferase 2 activity [GO:0043815] (molecular function) Also known as: 5'-phosphoribosylglycinamide transformylase 2, formate-dependent GAR transformylase activity, GAR transformylase 2, GART 2 References: PMID:8117714 Sources: RHEA:24829 Relationships: is a type of acid-ammonia (or amide) ligase activity [GO:0016880] Definition: Catalysis of the reaction: ATP + formate + N1-(5-phospho-beta-D-ribosyl)glycinamide = ADP + H+ + N2-formyl-N1-(5-phospho-beta-D-ribosyl)glycinamide + phosphate.